{
  "gene_name": "Ribonuclease inhibitor",
  "gene_symbol": "RNH1",
  "gene": "UniProtKB:P13489",
  "term_id": "GO:0008428",
  "term_label": "ribonuclease inhibitor activity"
}